{
  "gene": "UniProtKB:Q8N8R7",
  "gene_symbol": "ARL14EP",
  "term_label": "Unknown biological process",
  "gene_name": "ARL14 effector protein",
  "term_id": "UNKNOWN:0002"
}